{
  "term_id": "GO:0020037",
  "term_label": "heme binding",
  "gene": "UniProtKB:O43169",
  "gene_symbol": "CYB5B",
  "gene_name": "Cytochrome b5 type B"
}